protein localization to lateral cortical node [GO:1903360] (biological process) Relationships: is a type of protein localization to cell cortex [GO:0072697] Definition: A process in which a protein is transported to, or maintained in, a location within a lateral cortical node. References: PMID:25009287 Sources: GOC:TermGenie, GO_REF:0000087 Also known as: protein localisation in lateral cortical node, protein localisation to lateral cortical node, protein localization in lateral cortical node